{
  "gene": "UniProtKB:P57735",
  "gene_name": "Ras-related protein Rab-25",
  "gene_symbol": "RAB25",
  "term_label": "GTPase activity",
  "term_id": "GO:0003924"
}